7,8-dihydromonapterin aldolase activity [GO:0102083] (MF) References: PMID:15107504 Sources: GOC:pz Relationships: is a type of aldehyde-lyase activity [GO:0016832] Definition: Catalysis of the reaction: 7,8-dihydromonapterin = glycolaldehyde + 2-amino-6-(hydroxymethyl)-7,8-dihydropteridin-4-ol.